{
  "term_id": "GO:0019722",
  "gene_symbol": "P2RY11",
  "gene_name": "P2Y purinoceptor 11",
  "gene": "UniProtKB:Q96G91",
  "term_label": "calcium-mediated signaling"
}